{
  "term_id": "GO:0005634",
  "term_label": "nucleus",
  "gene": "UniProtKB:P53805",
  "gene_symbol": "RCAN1",
  "gene_name": "Calcipressin-1"
}